{
  "gene": "UniProtKB:Q96G28",
  "gene_name": "Cilia- and flagella-associated protein 36",
  "term_label": "Unknown molecular function",
  "term_id": "UNKNOWN:0001",
  "gene_symbol": "CFAP36"
}